{
  "term_label": "vesicle-mediated transport",
  "gene_symbol": "ARFGEF1",
  "gene": "UniProtKB:Q9Y6D6",
  "gene_name": "Brefeldin A-inhibited guanine nucleotide-exchange protein 1",
  "term_id": "GO:0016192"
}